{
  "term_id": "GO:0042088",
  "term_label": "T-helper 1 type immune response",
  "gene": "UniProtKB:Q14116",
  "gene_symbol": "IL18",
  "gene_name": "Interleukin-18"
}